glucan exo-1,3-beta-glucosidase activity [GO:0004338] (molecular function) Relationships: is a type of GO:0008422 Sources: EC:3.2.1.58 Definition: Catalysis of the successive hydrolysis of beta-D-glucose units from the non-reducing ends of (1->3)-beta-D-glucans, releasing alpha-glucose. Also known as: 1,3-beta-glucan glucohydrolase activity, glucan 1,3-beta-glucosidase activity, beta-1,3-glucan exo-hydrolase activity, exo (1->3)-beta-glucanase activity, exo-1,3-beta-D-glucanase activity, exo-1,3-beta-glucanase activity, exo-1,3-beta-glucosidase activity, exo-beta-(1->3)-D-glucanase activity, exo-beta-(1->3)-glucanohydrolase activity, exo-beta-1,3-D-glucanase activity, exo-beta-1,3-glucanase activity